{
  "gene_symbol": "SMPD2",
  "term_id": "GO:0006684",
  "term_label": "sphingomyelin metabolic process",
  "gene": "UniProtKB:O60906",
  "gene_name": "Sphingomyelin phosphodiesterase 2"
}